{
  "gene_symbol": "ADO",
  "gene": "UniProtKB:Q96SZ5",
  "gene_name": "2-aminoethanethiol dioxygenase",
  "term_id": "UNKNOWN:0002",
  "term_label": "Unknown biological process"
}